{
  "term_id": "GO:0006388",
  "gene": "UniProtKB:Q92989",
  "gene_symbol": "CLP1",
  "gene_name": "Polyribonucleotide 5'-hydroxyl-kinase Clp1",
  "term_label": "tRNA splicing, via endonucleolytic cleavage and ligation"
}